{
  "gene": "UniProtKB:Q8IXK0",
  "gene_name": "Polyhomeotic-like protein 2",
  "term_label": "negative regulation of DNA-templated transcription",
  "term_id": "GO:0045892",
  "gene_symbol": "PHC2"
}